{
  "gene_symbol": "IRAK1",
  "gene_name": "Interleukin-1 receptor-associated kinase 1",
  "gene": "UniProtKB:P51617",
  "term_id": "GO:0035556",
  "term_label": "intracellular signal transduction"
}